coenzyme F420 hydrogenase activity [GO:0050454] (molecular function) Also known as: 8-hydroxy-5-deazaflavin-reducing hydrogenase activity, F420-reducing hydrogenase activity, coenzyme F420-dependent hydrogenase activity, hydrogen:coenzyme F420 oxidoreductase activity Definition: Catalysis of the reaction: coenzyme F420 + H(2) + H+ = reduced coenzyme F420. Sources: EC:1.12.98.1, RHEA:23760 Relationships: is a type of oxidoreductase activity, acting on hydrogen as donor, with other known acceptors [GO:0046995]